{
  "term_label": "Unknown biological process",
  "gene": "UniProtKB:Q68D91",
  "gene_name": "Acyl-coenzyme A thioesterase MBLAC2",
  "term_id": "UNKNOWN:0002",
  "gene_symbol": "MBLAC2"
}